{
  "gene": "UniProtKB:Q16627",
  "term_label": "cell chemotaxis",
  "gene_symbol": "CCL14",
  "term_id": "GO:0060326",
  "gene_name": "C-C motif chemokine 14"
}